dUTP metabolic process [GO:0046080] (biological process) Subtypes: dUTP biosynthetic process [GO:0006229], GO:0046081 Also known as: dUTP metabolism Sources: GOC:go_curators Definition: The chemical reactions and pathways involving dUTP, deoxyuridine (5'-)triphosphate. Relationships: is a type of GO:0009211; is a type of pyrimidine deoxyribonucleotide metabolic process [GO:0009219]